{
  "term_id": "GO:0004197",
  "gene_name": "Caspase-9",
  "gene": "UniProtKB:P55211",
  "term_label": "cysteine-type endopeptidase activity",
  "gene_symbol": "CASP9"
}